{
  "gene_name": "Probable G-protein coupled receptor 146",
  "term_label": "Unknown cellular component",
  "gene": "UniProtKB:Q96CH1",
  "term_id": "UNKNOWN:0003",
  "gene_symbol": "GPR146"
}